{
  "gene_symbol": "RAD1",
  "term_label": "checkpoint clamp complex",
  "term_id": "GO:0030896",
  "gene_name": "Cell cycle checkpoint protein RAD1",
  "gene": "UniProtKB:O60671"
}